mRNA splice site recognition [GO:0006376] (biological process) Also known as: spliceosomal E complex biosynthesis, spliceosomal E complex formation, spliceosomal commitment complex biosynthesis, spliceosomal commitment complex formation Sources: GOC:krc, ISBN:0879695897 Relationships: is a type of GO:0022618; is part of spliceosomal complex assembly [GO:0000245] Definition: Selection of a splice site by components of the assembling spliceosome. Subtypes: mRNA 3'-splice site recognition [GO:0000389], mRNA 5'-splice site recognition [GO:0000395]